{
  "term_label": "RNA polymerase II transcription regulatory region sequence-specific DNA binding",
  "gene": "UniProtKB:Q9C0F3",
  "term_id": "GO:0000977",
  "gene_symbol": "ZNF436",
  "gene_name": "Zinc finger protein 436"
}